CDP-4-dehydro-6-deoxyglucose reductase activity [GO:0047099] (molecular function) Relationships: is a type of GO:0016726 Sources: EC:1.17.1.1, MetaCyc:1.17.1.1-RXN Also known as: CDP-4-dehydro-3,6-dideoxy-D-glucose:NAD(P)+ 3-oxidoreductase activity, CDP-4-keto-6-deoxy-D-glucose-3-dehydrogenase system activity, CDP-4-keto-6-deoxyglucose reductase activity, CDP-4-keto-deoxy-glucose reductase activity, NAD(P)H:CDP-4-keto-6-deoxy-D-glucose oxidoreductase activity, cytidine diphosphate 4-keto-6-deoxy-D-glucose-3-dehydrogenase activity, cytidine diphospho-4-keto-6-deoxy-D-glucose reductase activity Definition: Catalysis of the reaction: H2O + NAD(P)+ + CDP-4-dehydro-3,6-dideoxy-D-glucose = NAD(P)H + CDP-4-dehydro-6-deoxy-D-glucose.